{
  "gene": "UniProtKB:P08887",
  "term_label": "interleukin-6 binding",
  "term_id": "GO:0019981",
  "gene_name": "Interleukin-6 receptor subunit alpha",
  "gene_symbol": "IL6R"
}